{
  "gene_symbol": "TAPBPL",
  "gene": "UniProtKB:Q9BX59",
  "term_label": "MHC class I peptide loading complex",
  "term_id": "GO:0042824",
  "gene_name": "Tapasin-related protein"
}